{
  "gene_symbol": "PPY",
  "gene": "UniProtKB:P01298",
  "term_label": "neuropeptide Y receptor binding",
  "term_id": "GO:0031841",
  "gene_name": "Pancreatic polypeptide prohormone"
}